regulation of paraxial mesodermal cell fate determination [GO:0048345] (biological process) Subtypes: GO:0048346, negative regulation of paraxial mesodermal cell fate determination [GO:0048347] Relationships: is a type of regulation of mesodermal cell fate determination [GO:0048334]; regulates GO:0048344 Sources: GOC:dgh Definition: Any process that modulates the frequency, rate or extent of paraxial mesoderm cell fate determination.